{
  "term_id": "UNKNOWN:0003",
  "gene_name": "Coiled-coil domain-containing protein 183",
  "term_label": "Unknown cellular component",
  "gene_symbol": "CCDC183",
  "gene": "UniProtKB:Q5T5S1"
}